{
  "term_label": "fumarate transport",
  "gene_name": "Solute carrier family 13 member 2",
  "term_id": "GO:0015741",
  "gene_symbol": "SLC13A2",
  "gene": "UniProtKB:Q13183"
}